{
  "term_label": "nucleus",
  "gene_name": "Translation machinery-associated protein 16",
  "term_id": "GO:0005634",
  "gene_symbol": "TMA16",
  "gene": "UniProtKB:Q96EY4"
}